{
  "gene_name": "Sphingosine 1-phosphate receptor 3",
  "gene_symbol": "S1PR3",
  "term_label": "cytoplasm",
  "gene": "UniProtKB:Q99500",
  "term_id": "GO:0005737"
}